{
  "term_label": "Unknown cellular component",
  "term_id": "UNKNOWN:0003",
  "gene_symbol": "FAM83A",
  "gene_name": "Protein FAM83A",
  "gene": "UniProtKB:Q86UY5"
}